{
  "term_id": "GO:0007399",
  "gene": "UniProtKB:P78357",
  "gene_symbol": "CNTNAP1",
  "gene_name": "Contactin-associated protein 1",
  "term_label": "nervous system development"
}